{
  "gene": "UniProtKB:Q5GH77",
  "term_id": "UNKNOWN:0001",
  "term_label": "Unknown molecular function",
  "gene_name": "XK-related protein 3",
  "gene_symbol": "XKR3"
}